heart field specification [GO:0003128] (biological process) Sources: GOC:mtg_heart Definition: The process that results in the delineation of a specific region of the lateral mesoderm into the area in which the heart will develop. Relationships: is a type of GO:0010092; is part of heart formation [GO:0060914] Subtypes: GO:0003138, secondary heart field specification [GO:0003139] Regulation: positively regulated by heart induction [GO:0003129]